{
  "gene_symbol": "ITGAM",
  "term_label": "cell-cell adhesion",
  "term_id": "GO:0098609",
  "gene_name": "Integrin alpha-M",
  "gene": "UniProtKB:P11215"
}